amylin receptor 3 signaling pathway [GO:0150061] (biological process) Relationships: is a type of amylin receptor signaling pathway [GO:0097647] Also known as: AMY3 signaling pathway Definition: The series of molecular signals initiated by an extracellular amylin, or another ligand, combining with an amylin receptor 3 (AMY3), a G protein-coupled receptor complex, on the surface of the target cell. The AMY3 signaling pathway can also be initiated by the amyloid-beta complex. AMY3 signaling results in increased import of calcium ions into the cytosol across plasma membrane, increased phosphorylation of ERK1/2, Act, and a PKA regulatory subunit II, as well as increased expression of cFos. References: PMID:22500019 Sources: GOC:aruk, GOC:bc